{
  "term_id": "GO:0007224",
  "term_label": "smoothened signaling pathway",
  "gene_name": "Protein smoothened",
  "gene": "UniProtKB:Q99835",
  "gene_symbol": "SMO"
}